egg coat formation [GO:0035803] (biological process) Relationships: is a type of cellular process involved in reproduction in multicellular organism [GO:0022412]; BFO_0000050 oogenesis [GO:0048477] Definition: Construction of an egg coat, a specialized extracellular matrix that surrounds the ovum of animals. The egg coat provides structural support and can play an essential role in oogenesis, fertilization and early development. Also known as: VE formation, ZP assembly, vitelline envelope formation, zona pellucida assembly Subtypes: vitelline membrane formation [GO:0030704] References: PMID:16944418, PMID:17163408 Sources: GOC:bf, GOC:sart, GOC:yaf